{
  "term_id": "UNKNOWN:0001",
  "gene_name": "Arginine_serine-rich protein PNISR",
  "gene": "UniProtKB:Q8TF01",
  "term_label": "Unknown molecular function",
  "gene_symbol": "PNISR"
}